alpha-keto amide reductase activity [GO:0051268] (molecular function) Definition: Catalysis of the reaction: alpha-keto amide + 2 H+ (from donor) = (R)-hydroxy amide. Alpha-keto amides are of the form R-CO-CONH2, where R may be aromatic or aliphatic. References: PMID:15564669 Sources: GOC:ai Relationships: is a type of GO:0016903